metabolic compound salvage [GO:0043094] (biological process) Definition: Any process which produces a useful metabolic compound from derivatives of it without de novo synthesis, as carried out by individual cells. Sources: GOC:mlg Relationships: is a type of biosynthetic process [GO:0009058] Subtypes: pyrimidine-containing compound salvage [GO:0008655], pyridoxal 5'-phosphate salvage [GO:0009443], GO:0009853, oxidative photosynthetic carbon pathway [GO:0009854], phytol salvage [GO:0033307], GDP-L-fucose salvage [GO:0042352], GO:0043101, amino acid salvage [GO:0043102], nucleotide salvage [GO:0043173], GO:0043174